{
  "term_label": "formation of translation preinitiation complex",
  "gene": "UniProtKB:P41091",
  "term_id": "GO:0001731",
  "gene_name": "Eukaryotic translation initiation factor 2 subunit 3",
  "gene_symbol": "EIF2S3"
}